{
  "gene_name": "Activin receptor type-2A",
  "gene_symbol": "ACVR2A",
  "term_label": "plasma membrane",
  "gene": "UniProtKB:P27037",
  "term_id": "GO:0005886"
}